{
  "gene": "UniProtKB:P14416",
  "term_label": "phospholipase C-activating dopamine receptor signaling pathway",
  "gene_name": "D(2) dopamine receptor",
  "gene_symbol": "DRD2",
  "term_id": "GO:0060158"
}